{
  "term_label": "glutathione metabolic process",
  "gene_name": "Glutathione S-transferase Mu 1",
  "gene_symbol": "GSTM1",
  "term_id": "GO:0006749",
  "gene": "UniProtKB:P09488"
}